{
  "gene_symbol": "ARHGAP33",
  "gene_name": "Rho GTPase-activating protein 33",
  "term_id": "GO:0007264",
  "gene": "UniProtKB:O14559",
  "term_label": "small GTPase-mediated signal transduction"
}